{
  "term_label": "positive regulation of transcription by RNA polymerase II",
  "gene_name": "Transcription factor GATA-4",
  "term_id": "GO:0045944",
  "gene": "UniProtKB:P43694",
  "gene_symbol": "GATA4"
}